DNA strand elongation involved in DNA replication [GO:0006271] (biological process) Subtypes: leading strand elongation [GO:0006272], lagging strand elongation [GO:0006273], GO:1902296 Definition: The process in which an existing DNA strand is extended by activities including the addition of nucleotides to the 3' end of the strand, complementary to an existing template, as part of DNA replication. Sources: GOC:mah, ISBN:071673706X, ISBN:0815316194 Also known as: DNA replication elongation, DNA strand elongation during DNA replication Relationships: is a type of DNA strand elongation [GO:0022616]; is part of DNA-templated DNA replication [GO:0006261]; has part DNA synthesis involved in DNA replication [GO:0090592]